{
  "gene_symbol": "FAM167B",
  "gene_name": "Protein FAM167B",
  "term_label": "Unknown molecular function",
  "term_id": "UNKNOWN:0001",
  "gene": "UniProtKB:Q9BTA0"
}